pyruvate oxidase activity [GO:0047112] (molecular function) Definition: Catalysis of the reaction: H+ + O2 + phosphate + pyruvate = acetyl phosphate + CO2 + H2O2. Also known as: phosphate-dependent pyruvate oxidase activity, pyruvate:oxygen 2-oxidoreductase (phosphorylating), pyruvic oxidase activity Sources: RHEA:20848 Relationships: is a type of oxidoreductase activity, acting on the aldehyde or oxo group of donors, oxygen as acceptor [GO:0016623]